{
  "term_id": "GO:0005886",
  "gene_symbol": "OR2W6P",
  "gene_name": "Putative olfactory receptor 2W6",
  "term_label": "plasma membrane",
  "gene": "UniProtKB:Q8NHA6"
}